{
  "gene_name": "T cell receptor alpha joining 26 (Fragment)",
  "term_id": "UNKNOWN:0003",
  "gene_symbol": "TRAJ26",
  "term_label": "Unknown cellular component",
  "gene": "UniProtKB:A0A075B6V7"
}